positive regulation of acute inflammatory response to antigenic stimulus [GO:0002866] (biological process) Subtypes: positive regulation of hypersensitivity [GO:0002885] Relationships: is a type of positive regulation of acute inflammatory response [GO:0002675]; is a type of positive regulation of inflammatory response to antigenic stimulus [GO:0002863]; is_a regulation of acute inflammatory response to antigenic stimulus [GO:0002864]; positively regulates acute inflammatory response to antigenic stimulus [GO:0002438] Also known as: up regulation of acute inflammatory response to antigenic stimulus, up-regulation of acute inflammatory response to antigenic stimulus, upregulation of acute inflammatory response to antigenic stimulus, activation of acute inflammatory response to antigenic stimulus, stimulation of acute inflammatory response to antigenic stimulus Sources: GOC:add Definition: Any process that activates or increases the frequency, rate, or extent of an acute inflammatory response to an antigenic stimulus.